ATP diphosphatase activity [GO:0047693] (molecular function) Definition: Catalysis of the reaction: ATP + H2O = AMP + H+ + diphosphate. Sources: RHEA:14245 Relationships: is a type of nucleoside triphosphate diphosphatase activity [GO:0047429] Also known as: ATP diphosphohydrolase, ATP diphosphohydrolase (diphosphate-forming), ATP pyrophosphatase activity, adenosine triphosphate pyrophosphatase activity